{
  "term_label": "regulation of cell migration",
  "gene": "UniProtKB:O95750",
  "gene_name": "Fibroblast growth factor 19",
  "term_id": "GO:0030334",
  "gene_symbol": "FGF19"
}